{
  "term_label": "DNA-binding transcription factor activity, RNA polymerase II-specific",
  "gene": "UniProtKB:Q8WV37",
  "gene_symbol": "ZNF480",
  "term_id": "GO:0000981",
  "gene_name": "Zinc finger protein 480"
}